{
  "gene_symbol": "PTGER4",
  "gene_name": "Prostaglandin E2 receptor EP4 subtype",
  "term_id": "GO:0007189",
  "gene": "UniProtKB:P35408",
  "term_label": "adenylate cyclase-activating G protein-coupled receptor signaling pathway"
}